{
  "gene": "UniProtKB:P49760",
  "gene_name": "Dual specificity protein kinase CLK2",
  "term_id": "GO:0004674",
  "gene_symbol": "CLK2",
  "term_label": "protein serine/threonine kinase activity"
}